{
  "gene": "UniProtKB:P16519",
  "term_id": "GO:0004252",
  "gene_name": "Neuroendocrine convertase 2",
  "term_label": "serine-type endopeptidase activity",
  "gene_symbol": "PCSK2"
}